{
  "gene_name": "SH3 domain-binding protein 4",
  "gene_symbol": "SH3BP4",
  "gene": "UniProtKB:Q9P0V3",
  "term_label": "Unknown molecular function",
  "term_id": "UNKNOWN:0001"
}